{
  "gene_name": "Cytoplasmic dynein 1 light intermediate chain 2",
  "term_label": "cytoplasmic dynein complex",
  "gene": "UniProtKB:O43237",
  "gene_symbol": "DYNC1LI2",
  "term_id": "GO:0005868"
}